{
  "gene_symbol": "GRID2",
  "term_id": "GO:0050804",
  "gene": "UniProtKB:O43424",
  "gene_name": "Glutamate receptor ionotropic, delta-2",
  "term_label": "modulation of chemical synaptic transmission"
}